{
  "gene": "UniProtKB:Q15878",
  "term_id": "GO:0098703",
  "gene_symbol": "CACNA1E",
  "term_label": "calcium ion import across plasma membrane",
  "gene_name": "Voltage-dependent R-type calcium channel subunit alpha-1E"
}